{
  "term_id": "GO:0005737",
  "gene": "UniProtKB:Q8WUQ7",
  "gene_name": "Splicing factor Cactin",
  "gene_symbol": "CACTIN",
  "term_label": "cytoplasm"
}